{
  "term_label": "ubiquitin protein ligase activity",
  "term_id": "GO:0061630",
  "gene_name": "E3 ubiquitin-protein ligase ARIH2",
  "gene_symbol": "ARIH2",
  "gene": "UniProtKB:O95376"
}